negative regulation of ATP-dependent activity [GO:0032780] (biological process) Relationships: is a type of regulation of ATP-dependent activity [GO:0043462]; is a type of negative regulation of molecular function [GO:0044092]; negatively regulates GO:0140657 Also known as: down regulation of ATPase activity, down-regulation of ATPase activity, downregulation of ATPase activity, negative regulation of ATPase activity, negative regulation of adenosinetriphosphatase activity, inhibition of ATPase activity Sources: GOC:mah Definition: Any process that stops or reduces the rate of an ATP-dependent activity. Subtypes: negative regulation of helicase activity [GO:0051097], GO:1901895, negative regulation of P-type sodium:potassium-exchanging transporter activity [GO:1903407], GO:1903611